cell adhesion molecule binding [GO:0050839] (molecular function) Definition: Binding to a cell adhesion molecule. Sources: GOC:ai Also known as: CAM binding, adhesive extracellular matrix constituent, cell adhesion molecule activity, cell adhesion receptor activity Relationships: is a type of protein binding [GO:0005515] Subtypes: GO:0005178, cadherin binding [GO:0045296], GO:0098631